{
  "term_label": "sodium ion import across plasma membrane",
  "gene": "UniProtKB:Q96T83",
  "gene_symbol": "SLC9A7",
  "gene_name": "Sodium_hydrogen exchanger 7",
  "term_id": "GO:0098719"
}